anterograde axonal transport of neurotransmitter receptor complex [GO:0140231] (biological process) Relationships: is a type of receptor localization to synapse [GO:0097120]; is a type of neurotransmitter receptor transport [GO:0099637]; is a type of anterograde axonal protein transport [GO:0099641] Definition: The directed movement of a neurotransmitter receptor complex along microtubules from the cell body toward the cell periphery in nerve cell axons. References: PMID:28680963